{
  "term_label": "eukaryotic translation initiation factor 3 complex",
  "gene_symbol": "EIF3B",
  "term_id": "GO:0005852",
  "gene": "UniProtKB:P55884",
  "gene_name": "Eukaryotic translation initiation factor 3 subunit B"
}